{
  "term_label": "plasma membrane",
  "gene": "UniProtKB:O60423",
  "gene_name": "Phospholipid-transporting ATPase IK",
  "term_id": "GO:0005886",
  "gene_symbol": "ATP8B3"
}